{
  "gene": "UniProtKB:O75309",
  "gene_name": "Cadherin-16",
  "term_label": "cell-cell adhesion",
  "gene_symbol": "CDH16",
  "term_id": "GO:0098609"
}